Edg-5 sphingosine 1-phosphate receptor binding [GO:0031758] (molecular function) Relationships: is a type of GO:0031753 Sources: GOC:mah, GOC:nln Definition: Binding to an Edg-5 sphingosine 1-phosphate receptor. Also known as: Edg-5 sphingosine 1-phosphate receptor ligand